{
  "term_id": "GO:0072344",
  "gene": "UniProtKB:Q15650",
  "gene_name": "Activating signal cointegrator 1",
  "gene_symbol": "TRIP4",
  "term_label": "rescue of stalled ribosome"
}